{
  "term_label": "Unknown molecular function",
  "gene": "UniProtKB:Q8N357",
  "gene_name": "Solute carrier family 35 member F6",
  "gene_symbol": "SLC35F6",
  "term_id": "UNKNOWN:0001"
}